ceramide phosphoethanolamine synthase activity [GO:0002950] (molecular function) References: PMID:25667419 Sources: EC:2.7.8.48 Relationships: is a type of GO:0016780 Definition: Catalysis of the reaction: an N-acyl-sphingoid base + CDP-ethanolamine = an N-acyl-sphingoid 1-phosphoethanolamine + CMP + H+.